{
  "gene": "UniProtKB:P07947",
  "term_label": "non-membrane spanning protein tyrosine kinase activity",
  "gene_symbol": "YES1",
  "gene_name": "Tyrosine-protein kinase Yes",
  "term_id": "GO:0004715"
}